{
  "gene_symbol": "Q71RC1",
  "gene_name": "PP13850",
  "gene": "UniProtKB:Q71RC1",
  "term_id": "UNKNOWN:0003",
  "term_label": "Unknown cellular component"
}